{
  "gene": "UniProtKB:P54277",
  "gene_name": "PMS1 protein homolog 1",
  "gene_symbol": "PMS1",
  "term_label": "mismatch repair complex",
  "term_id": "GO:0032300"
}